{
  "gene_symbol": "FLVCR1",
  "gene": "UniProtKB:Q9Y5Y0",
  "gene_name": "Heme transporter FLVCR1",
  "term_label": "heme export",
  "term_id": "GO:0097037"
}